{
  "gene_symbol": "A1L4Q6",
  "gene_name": "Putative uncharacterized protein FLJ41423",
  "gene": "UniProtKB:A1L4Q6",
  "term_label": "Unknown cellular component",
  "term_id": "UNKNOWN:0003"
}